{
  "term_label": "phosphatidylinositol-3-phosphate binding",
  "term_id": "GO:0032266",
  "gene": "UniProtKB:O60493",
  "gene_symbol": "SNX3",
  "gene_name": "Sorting nexin-3"
}